{
  "term_label": "oxidoreductase activity, acting on the CH-OH group of donors, NAD or NADP as acceptor",
  "gene_symbol": "SDR42E2",
  "term_id": "GO:0016616",
  "gene_name": "Putative short-chain dehydrogenase_reductase family 42E member 2",
  "gene": "UniProtKB:A6NKP2"
}